L-serine import across plasma membrane [GO:1903812] (biological process) Also known as: L-serine import into cell References: PMID:23895341 Sources: GOC:TermGenie, GO_REF:0000075 Definition: The directed movement of L-serine into a cell. Relationships: is a type of L-serine transport [GO:0015825]; is a type of serine import across plasma membrane [GO:0098718]; is a type of L-alpha-amino acid transmembrane transport [GO:1902475]